{
  "term_id": "GO:0045944",
  "gene_symbol": "HOXC4",
  "gene_name": "Homeobox protein Hox-C4",
  "gene": "UniProtKB:P09017",
  "term_label": "positive regulation of transcription by RNA polymerase II"
}